{
  "term_id": "GO:0006413",
  "gene": "UniProtKB:Q14232",
  "term_label": "translational initiation",
  "gene_name": "Translation initiation factor eIF-2B subunit alpha",
  "gene_symbol": "EIF2B1"
}